regulation of protein homotetramerization [GO:1901093] (biological process) Relationships: is a type of regulation of protein homooligomerization [GO:0032462]; is a type of regulation of protein tetramerization [GO:1901090]; regulates protein homotetramerization [GO:0051289] Subtypes: negative regulation of protein homotetramerization [GO:1901094], positive regulation of protein homotetramerization [GO:1901095] Sources: GOC:TermGenie, GOC:pm Definition: Any process that modulates the frequency, rate or extent of protein homotetramerization. Also known as: regulation of protein homotetramer assembly, regulation of protein homotetramer biosynthesis, regulation of protein homotetramer biosynthetic process, regulation of protein homotetramer formation